positive regulation of short-term synaptic potentiation [GO:1905514] (biological process) Definition: Any process that activates or increases the frequency, rate or extent of short-term synaptic potentiation. References: PMID:15470145 Sources: GOC:TermGenie, GOC:hjd, GO_REF:0000058 Also known as: positive regulation of synaptic facilitation, up regulation of short-term synaptic potentiation, up regulation of synaptic facilitation, up-regulation of short-term synaptic potentiation, up-regulation of synaptic facilitation, upregulation of short-term synaptic potentiation, upregulation of synaptic facilitation, activation of short-term synaptic potentiation, activation of synaptic facilitation Relationships: is a type of GO:0048518; is a type of regulation of short-term synaptic potentiation [GO:1905512]; positively regulates GO:1990926